{
  "gene_symbol": "TRAV27",
  "gene_name": "T cell receptor alpha variable 27",
  "gene": "UniProtKB:A0A087WT01",
  "term_label": "response to bacterium",
  "term_id": "GO:0009617"
}